{
  "gene": "UniProtKB:Q96Q45",
  "term_id": "GO:0060271",
  "gene_name": "Transmembrane protein 237",
  "term_label": "cilium assembly",
  "gene_symbol": "TMEM237"
}